{
  "gene": "UniProtKB:P08581",
  "gene_symbol": "MET",
  "gene_name": "Hepatocyte growth factor receptor",
  "term_id": "GO:0007169",
  "term_label": "cell surface receptor protein tyrosine kinase signaling pathway"
}